{
  "term_label": "Golgi membrane",
  "gene": "UniProtKB:Q9C0J1",
  "gene_name": "N-acetyllactosaminide beta-1,3-N-acetylglucosaminyltransferase 4",
  "term_id": "GO:0000139",
  "gene_symbol": "B3GNT4"
}